{
  "gene_symbol": "CDH9",
  "gene_name": "Cadherin-9",
  "term_label": "cadherin binding",
  "gene": "UniProtKB:Q9ULB4",
  "term_id": "GO:0045296"
}